{
  "gene": "UniProtKB:Q96LD4",
  "gene_name": "E3 ubiquitin-protein ligase TRIM47",
  "term_id": "UNKNOWN:0002",
  "gene_symbol": "TRIM47",
  "term_label": "Unknown biological process"
}